{
  "gene": "UniProtKB:P67870",
  "gene_symbol": "CSNK2B",
  "term_label": "Unknown biological process",
  "gene_name": "Casein kinase II subunit beta",
  "term_id": "UNKNOWN:0002"
}